valine dehydrogenase (NAD+) activity [GO:0043837] (molecular function) References: PMID:10612726, PMID:2803248 Definition: Catalysis of the reaction: L-valine + H2O + NAD+ = 3-methyl-2-oxobutanoate + NH3 + NADH. Relationships: is a type of GO:0016639 Also known as: valine dehydrogenase (NAD) activity, ValDH